{
  "gene": "UniProtKB:Q5SYC1",
  "gene_symbol": "CLVS2",
  "term_label": "clathrin-coated vesicle",
  "gene_name": "Clavesin-2",
  "term_id": "GO:0030136"
}